{
  "gene": "UniProtKB:P07202",
  "term_id": "GO:0005615",
  "gene_symbol": "TPO",
  "gene_name": "Thyroid peroxidase",
  "term_label": "extracellular space"
}